2-alpha-hydroxytaxane 2-O-benzoyltransferase activity [GO:0050642] (molecular function) Relationships: is a type of acyltransferase activity, transferring groups other than amino-acyl groups [GO:0016747] Also known as: 2a-hydroxytaxane 2-O-benzoyltransferase activity, 2-debenzoyl-7,13-diacetylbaccatin III-2-O-benzoyl transferase activity, 2alpha-hydroxytaxane 2-O-benzoyltransferase activity, benzoyl-CoA:taxan-2alpha-ol O-benzoyltransferase activity, benzoyl-CoA:taxane 2-alpha-O-benzoyltransferase activity, benzoyl-CoA:taxane 2alpha-O-benzoyltransferase activity Sources: RHEA:18741 Definition: Catalysis of the reaction: 10-deacetyl-2-debenzoylbaccatin III + benzoyl-CoA = 10-deacetylbaccatin III + CoA.